{
  "gene_name": "Calcium-dependent secretion activator 2",
  "gene": "UniProtKB:Q86UW7",
  "term_id": "UNKNOWN:0001",
  "gene_symbol": "CADPS2",
  "term_label": "Unknown molecular function"
}